platelet formation [GO:0030220] (biological process) Regulation: regulated by regulation of platelet formation [GO:1905219]; negatively regulated by negative regulation of platelet formation [GO:1905220]; positively regulated by positive regulation of platelet formation [GO:1905221] Sources: GOC:mah, ISBN:0815316194 Relationships: is a type of GO:0030099; is a type of GO:0048646; is part of GO:0036344 Also known as: platelet extrusion Definition: The process in which platelets bud from long processes extended by megakaryocytes.